{
  "gene_symbol": "ACADSB",
  "term_id": "GO:0003995",
  "gene": "UniProtKB:P45954",
  "gene_name": "Short_branched chain specific acyl-CoA dehydrogenase, mitochondrial",
  "term_label": "acyl-CoA dehydrogenase activity"
}